{
  "gene": "UniProtKB:Q8IV01",
  "term_id": "GO:0061891",
  "gene_symbol": "SYT12",
  "gene_name": "Synaptotagmin-12",
  "term_label": "calcium ion sensor activity"
}